{
  "gene_name": "CUB domain-containing protein 1",
  "gene_symbol": "CDCP1",
  "gene": "UniProtKB:Q9H5V8",
  "term_label": "Unknown cellular component",
  "term_id": "UNKNOWN:0003"
}